{
  "gene_symbol": "TNFSF8",
  "term_label": "CD8-positive, alpha-beta T cell differentiation",
  "gene": "UniProtKB:P32971",
  "term_id": "GO:0043374",
  "gene_name": "Tumor necrosis factor ligand superfamily member 8"
}